positive regulation of laminaritriose transport [GO:1900305] (biological process) Also known as: up regulation of laminaritriose transport, up-regulation of laminaritriose transport, upregulation of laminaritriose transport, activation of laminaritriose transport Sources: GOC:TermGenie, GOC:mengo_curators Relationships: is a type of positive regulation of transport [GO:0051050]; is a type of regulation of laminaritriose transport [GO:1900303]; positively regulates laminaritriose transport [GO:2001097] Definition: Any process that activates or increases the frequency, rate or extent of laminaritriose transport.